{
  "gene_name": "Beta_gamma crystallin domain-containing protein 1",
  "term_id": "UNKNOWN:0003",
  "gene": "UniProtKB:Q9Y4K1",
  "term_label": "Unknown cellular component",
  "gene_symbol": "CRYBG1"
}